{
  "gene": "UniProtKB:Q5T601",
  "term_label": "G protein-coupled receptor activity",
  "gene_symbol": "ADGRF1",
  "gene_name": "Adhesion G-protein coupled receptor F1",
  "term_id": "GO:0004930"
}